{
  "term_id": "UNKNOWN:0002",
  "gene_symbol": "DSCR9",
  "gene": "UniProtKB:P59020",
  "term_label": "Unknown biological process",
  "gene_name": "Down syndrome critical region protein 9"
}